{
  "gene_name": "Potassium voltage-gated channel subfamily E member 1",
  "gene": "UniProtKB:P15382",
  "term_id": "GO:0005251",
  "term_label": "delayed rectifier potassium channel activity",
  "gene_symbol": "KCNE1"
}